{
  "gene": "UniProtKB:Q13243",
  "gene_symbol": "SRSF5",
  "term_label": "regulation of alternative mRNA splicing, via spliceosome",
  "term_id": "GO:0000381",
  "gene_name": "Serine_arginine-rich splicing factor 5"
}